{
  "term_label": "Unknown biological process",
  "gene": "UniProtKB:Q9UIL1",
  "term_id": "UNKNOWN:0002",
  "gene_symbol": "SCOC",
  "gene_name": "Short coiled-coil protein"
}